sulcatone reductase activity [GO:0050491] (molecular function) Sources: EC:1.1.1.260, RHEA:24484 Relationships: is a type of oxidoreductase activity, acting on the CH-OH group of donors, NAD or NADP as acceptor [GO:0016616] Definition: Catalysis of the reaction: NAD+ + sulcatol = H+ + NADH + sulcatone. Also known as: sulcatol:NAD+ oxidoreductase activity